{
  "gene_name": "Proline-rich protein 20C",
  "term_label": "Unknown biological process",
  "gene": "UniProtKB:P86479",
  "term_id": "UNKNOWN:0002",
  "gene_symbol": "PRR20C"
}